{
  "gene_name": "Hedgehog-interacting protein",
  "term_label": "Unknown molecular function",
  "gene_symbol": "HHIP",
  "gene": "UniProtKB:Q96QV1",
  "term_id": "UNKNOWN:0001"
}